{
  "gene_symbol": "LIPN",
  "gene": "UniProtKB:Q5VXI9",
  "term_label": "Unknown cellular component",
  "gene_name": "Lipase member N",
  "term_id": "UNKNOWN:0003"
}